{
  "gene_name": "Thy-1 membrane glycoprotein",
  "term_label": "external side of plasma membrane",
  "term_id": "GO:0009897",
  "gene": "UniProtKB:P04216",
  "gene_symbol": "THY1"
}